{
  "gene_name": "Nipped-B-like protein",
  "term_label": "embryonic viscerocranium morphogenesis",
  "term_id": "GO:0048703",
  "gene_symbol": "NIPBL",
  "gene": "UniProtKB:Q6KC79"
}